pyrimidine nucleobase fermentation [GO:0043466] (biological process) Definition: The anaerobic conversion of pyrimidine nucleobases, yielding energy in the form of ATP. Sources: GOC:jl Also known as: pyrimidine base fermentation, pyrimidine fermentation Relationships: is a type of fermentation [GO:0006113]; is a type of pyrimidine nucleobase catabolic process [GO:0006208]